acidocalcisome lumen [GO:0033985] (cellular component) Sources: GOC:mah Definition: The volume enclosed by the membranes of an acidocalcisome. Relationships: is a type of intracellular organelle lumen [GO:0070013]; is part of acidocalcisome [GO:0020022]